{
  "gene": "UniProtKB:O95479",
  "gene_name": "GDH_6PGL endoplasmic bifunctional protein",
  "gene_symbol": "H6PD",
  "term_id": "GO:0004345",
  "term_label": "glucose-6-phosphate dehydrogenase activity"
}